symbiont-mediated suppression of host programmed cell death [GO:0052041] (BP) Definition: A process in which a symbiont inhibits or disrupts the normal execution of host programmed cell death, leading to a decrease in the frequency, rate or extent of programmed cell death in the host cell. The host is defined as the larger of the organisms involved in a symbiotic interaction. Sources: GOC:curators Also known as: down regulation by symbiont of host programmed cell death, down-regulation by symbiont of host programmed cell death, downregulation by symbiont of host programmed cell death, inhibition of host programmed cell death, negative regulation by symbiont of host programmed cell death, suppression by symbiont of host PCD, suppression by symbiont of host programmed cell death, inhibition by symbiont of host programmed cell death Relationships: is a type of symbiont-mediated perturbation of host programmed cell death [GO:0052040] Subtypes: symbiont-mediated suppression of host apoptosis [GO:0033668]